{
  "gene_symbol": "AR",
  "term_id": "GO:0000785",
  "gene_name": "Androgen receptor",
  "term_label": "chromatin",
  "gene": "UniProtKB:P10275"
}